{
  "gene_symbol": "SYNDIG1",
  "gene_name": "Synapse differentiation-inducing gene protein 1",
  "term_label": "positive regulation of synapse assembly",
  "term_id": "GO:0051965",
  "gene": "UniProtKB:Q9H7V2"
}